tRNA-uracil-4 sulfurtransferase activity [GO:0140741] (molecular function) Definition: Catalyzes the reaction: ATP + [ThiI sulfur-carrier protein]-S-sulfanyl-L-cysteine + uracil in tRNA + 2 reduced ferredoxin [iron-sulfur] cluster = AMP + diphosphate + 4-thiouracil in tRNA + [ThiI sulfur-carrier protein]-L-cysteine + 2 oxidized ferredoxin [iron-sulfur] cluster. References: PMID:27791189, PMID:5541999 Sources: RHEA:24176 Also known as: tRNA U4 sulfurtransferase, tRNA uracil 4 sulfurtransferase, tRNA uracil 4-sulfurtransferase Relationships: is a type of sulfurtransferase activity [GO:0016783]; is a type of GO:0140101